{
  "term_id": "GO:0007186",
  "gene": "UniProtKB:Q9BY21",
  "gene_name": "G-protein coupled receptor 87",
  "term_label": "G protein-coupled receptor signaling pathway",
  "gene_symbol": "GPR87"
}